{
  "gene": "UniProtKB:Q14940",
  "term_id": "GO:0098719",
  "gene_symbol": "SLC9A5",
  "gene_name": "Sodium_hydrogen exchanger 5",
  "term_label": "sodium ion import across plasma membrane"
}